{
  "gene_symbol": "POF1B",
  "term_label": "actin filament",
  "term_id": "GO:0005884",
  "gene": "UniProtKB:Q8WVV4",
  "gene_name": "Protein POF1B"
}